lipopolysaccharide N-acetylglucosaminyltransferase activity [GO:0008917] (molecular function) Relationships: is a type of acetylglucosaminyltransferase activity [GO:0008375]; is part of lipopolysaccharide biosynthetic process [GO:0009103] Sources: EC:2.4.1.56, GOC:mr Also known as: LPS N-acetylglucosaminyltransferase activity, UDP-N-acetyl-D-glucosamine:lipopolysaccharide N-acetyl-D-glucosaminyltransferase activity, UDP-N-acetylglucosamine-lipopolysaccharide N-acetylglucosaminyltransferase activity, uridine diphosphoacetylglucosamine-lipopolysaccharide acetylglucosaminyltransferase activity Definition: Catalysis of the reaction: UDP-N-acetyl-D-glucosamine + lipopolysaccharide = UDP + N-acetyl-D-glucosaminyl-lipopolysaccharide.